{
  "gene": "UniProtKB:Q8TF72",
  "gene_symbol": "SHROOM3",
  "gene_name": "Protein Shroom3",
  "term_id": "GO:0007015",
  "term_label": "actin filament organization"
}